{
  "gene_name": "Pre-B-cell leukemia transcription factor 1",
  "gene_symbol": "PBX1",
  "term_label": "RNA polymerase II cis-regulatory region sequence-specific DNA binding",
  "term_id": "GO:0000978",
  "gene": "UniProtKB:P40424"
}